mesonephros morphogenesis [GO:0061206] (biological process) Definition: The process in which the anatomical structures of the mesonephros are generated and organized. Also known as: Wolffian body morphogenesis Relationships: is a type of GO:0060993; is part of mesonephros development [GO:0001823] Sources: GOC:mtg_kidney_jan10